{
  "term_id": "GO:0016887",
  "gene": "UniProtKB:Q02241",
  "gene_name": "Kinesin-like protein KIF23",
  "gene_symbol": "KIF23",
  "term_label": "ATP hydrolysis activity"
}